long-chain fatty-acyl-CoA metabolic process [GO:0035336] (biological process) Also known as: long-chain fatty acyl CoA metabolic process, long-chain fatty acyl-CoA metabolism Definition: The chemical reactions and pathways involving long-chain fatty-acyl-CoAs, any derivative of coenzyme A in which the sulfhydryl group is in a thioester linkage with a long-chain fatty-acyl group. A long-chain fatty acid has an aliphatic tail containing 13 to 22 carbons. Note: While there is not universal consensus on the lengths of short-, medium-, long- and very-long-chain fatty acids, the GO uses the definitions in ChEBI (see CHEBI:26666, CHEBI:59554, CHEBI:15904 and CHEBI:27283). Sources: ISBN:0198506732 Relationships: is_a fatty-acyl-CoA metabolic process [GO:0035337] Subtypes: long-chain fatty-acyl-CoA biosynthetic process [GO:0035338], long-chain fatty-acyl-CoA catabolic process [GO:0036116]